alphaV-beta3 integrin-EGFR complex [GO:0071125] (cellular component) Definition: A protein complex that consists of an alphaV-beta3 integrin complex bound to epidermal growth factor receptor. Also known as: ITGAV-ITGB3-EGFR complex References: PMID:15834425 Relationships: is a type of plasma membrane protein complex [GO:0098797]